{
  "gene_name": "Cytosolic non-specific dipeptidase",
  "gene_symbol": "CNDP2",
  "term_label": "cytosol",
  "term_id": "GO:0005829",
  "gene": "UniProtKB:Q96KP4"
}